{
  "term_id": "GO:0005737",
  "gene_name": "Tubulin beta chain",
  "gene": "UniProtKB:P07437",
  "gene_symbol": "TUBB",
  "term_label": "cytoplasm"
}